{
  "gene": "UniProtKB:P32247",
  "term_label": "neuropeptide receptor activity",
  "gene_symbol": "BRS3",
  "term_id": "GO:0008188",
  "gene_name": "Bombesin receptor subtype-3"
}